{
  "term_id": "GO:0001707",
  "term_label": "mesoderm formation",
  "gene_name": "Eomesodermin homolog",
  "gene_symbol": "EOMES",
  "gene": "UniProtKB:O95936"
}